{
  "term_label": "semaphorin-plexin signaling pathway",
  "gene_symbol": "PLXNB1",
  "term_id": "GO:0071526",
  "gene_name": "Plexin-B1",
  "gene": "UniProtKB:O43157"
}